transcription corepressor activity [GO:0003714] (molecular function) References: PMID:10213677, PMID:16858867 Sources: GOC:txnOH-2018 Relationships: is a type of GO:0003712; is part of GO:0045892 Definition: A transcription coregulator activity that represses or decreases the transcription of specific gene sets via binding to a DNA-binding transcription factor at a specific genomic locus, either on its own or as part of a complex. Corepressors often act by altering chromatin structure and modifications. For example, one class of transcription corepressors modifies chromatin structure through covalent modification of histones. A second class remodels the conformation of chromatin in an ATP-dependent fashion. A third class modulates interactions of DNA-bound DNA-binding transcription factors with other transcription coregulators. Subtypes: GO:0016989 Note: For usage guidance, see comment in GO:0003712 ; transcription coregulator activity. Also known as: transcription co-repressor activity, RNA polymerase II transcription co-repressor activity, RNA polymerase II transcription corepressor activity